{
  "gene_symbol": "MS4A6A",
  "term_label": "plasma membrane",
  "gene_name": "Membrane-spanning 4-domains subfamily A member 6A",
  "term_id": "GO:0005886",
  "gene": "UniProtKB:Q9H2W1"
}